{
  "term_id": "GO:0005524",
  "gene": "UniProtKB:Q9Y3D8",
  "term_label": "ATP binding",
  "gene_name": "Adenylate kinase isoenzyme 6",
  "gene_symbol": "AK6"
}